9,9'-di-cis-zeta-carotene desaturase activity [GO:0016719] (MF) Relationships: is a type of oxidoreductase activity, acting on the CH-CH group of donors, quinone or related compound as acceptor [GO:0016635] Also known as: carotene 7,8-desaturase activity, carotene,hydrogen-donor:oxygen oxidoreductase activity, zeta-carotene desaturase activity Sources: RHEA:30955 Definition: Catalysis of the reaction: 9,9'-di-cis-zeta-carotene + 2 a quinone = 7,7',9,9'-tetra-cis-lycopene + 2 a quinol.